{
  "gene": "UniProtKB:Q92508",
  "gene_name": "Piezo-type mechanosensitive ion channel component 1",
  "gene_symbol": "PIEZO1",
  "term_id": "GO:0140135",
  "term_label": "mechanosensitive monoatomic cation channel activity"
}